{
  "gene_symbol": "OR2H1",
  "term_id": "GO:0050911",
  "gene_name": "Olfactory receptor 2H1",
  "term_label": "detection of chemical stimulus involved in sensory perception of smell",
  "gene": "UniProtKB:Q9GZK4"
}